{
  "gene_name": "Eyes absent homolog 1",
  "gene": "UniProtKB:Q99502",
  "gene_symbol": "EYA1",
  "term_label": "nucleus",
  "term_id": "GO:0005634"
}